acyl-lipid omega-6 desaturase (cytochrome b5) activity [GO:0050184] (molecular function) Sources: RHEA:46332 Also known as: 1-16:0-2-18:1-phosphatidylcholine desaturase activity, 1-18:1-2-18:2-phosphatidylcholine desaturase activity, 1-18:1-2-18:2-phosphatidylcholine synthase activity, 1-18:1-2-18:3-phosphatidylcholinedesaturase activity, 1-18:2-2-18:1-phosphatidylcholine desaturase activity (SN2-18:2 forming), 1-acyl-2-oleoyl-sn-glycero-3-phosphocholine:NAD+ delta12-oxidoreductase activity, linoleate synthase activity, oleate desaturase activity, oleoyl-CoA desaturase activity, oleoylphosphatidylcholine desaturase activity, phosphatidylcholine desaturase activity Definition: Catalysis of the reaction: a (9Z)-octadecenoyl-containing glycerolipid + 2 Fe(II)-[cytochrome b5] + 2 H+ + O2 = a (9Z,12Z)-octadecadienoyl-containing glycerolipid + 2 Fe(III)-[cytochrome b5] + 2 H2O. Relationships: is a type of oxidoreductase activity, acting on paired donors, with oxidation of a pair of donors resulting in the reduction of molecular oxygen to two molecules of water [GO:0016717]